mitotic actomyosin contractile ring, distal actin filament layer [GO:0120106] (cellular component) References: PMID:28914606 Sources: GOC:krc, GOC:vw Relationships: is_a cellular anatomical structure [GO:0110165]; is part of mitotic actomyosin contractile ring [GO:0110085] Definition: The region of the mitotic actomyosin ring containing actin filaments and cross linkers, myosin motors, and connections to the plasma membrane through the intermediate layer. It is further from the plasma membrane than the intermediate layer which it is adjacent to. Also known as: actomyosin contractile ring, distal actin filament layer